{
  "gene_symbol": "RIC8A",
  "gene_name": "Synembryn-A",
  "gene": "UniProtKB:Q9NPQ8",
  "term_id": "GO:0007186",
  "term_label": "G protein-coupled receptor signaling pathway"
}